G protein-coupled receptor binding [GO:0001664] (molecular function) Definition: Binding to a G protein-coupled receptor. Subtypes: frizzled binding [GO:0005109], smoothened binding [GO:0005119], GO:0031531, opioid receptor binding [GO:0031628], adenosine receptor binding [GO:0031685], adrenergic receptor binding [GO:0031690], adrenomedullin receptor binding [GO:0031700], GO:0031701, bradykinin receptor binding [GO:0031711], C5a anaphylatoxin chemotactic receptor binding [GO:0031714], GO:0031716, cannabinoid receptor binding [GO:0031717], cysteinyl leukotriene receptor binding [GO:0031745], GO:0031753, fMet-Leu-Phe receptor binding [GO:0031761], follicle-stimulating hormone receptor binding [GO:0031762], gastric inhibitory polypeptide receptor binding [GO:0031767], ghrelin receptor binding [GO:0031768], GO:0031769, leukotriene receptor binding [GO:0031774], lutropin-choriogonadotropic hormone receptor binding [GO:0031775], melatonin receptor binding [GO:0031784], motilin receptor binding [GO:0031788], GO:0031789, GO:0031795, G protein-coupled histamine receptor binding [GO:0031806], G protein-coupled nucleotide receptor binding [GO:0031811], G protein-coupled serotonin receptor binding [GO:0031821], olfactory receptor binding [GO:0031849], oxytocin receptor binding [GO:0031855], parathyroid hormone receptor binding [GO:0031856], platelet activating factor receptor binding [GO:0031859], prostanoid receptor binding [GO:0031862], proteinase activated receptor binding [GO:0031871], GO:0031876, taste receptor binding [GO:0031883], urotensin receptor binding [GO:0031889], vasopressin receptor binding [GO:0031893], G protein-coupled glutamate receptor binding [GO:0035256], chemokine receptor binding [GO:0042379], GO:0050780, alpha-latrotoxin receptor binding [GO:0061761], GO:0071855 Relationships: is a type of signaling receptor binding [GO:0005102] Also known as: G protein coupled receptor binding, G-protein coupled receptor binding, G protein coupled receptor ligand, G-protein-coupled receptor ligand Sources: GOC:ceb, GOC:dph